{
  "gene_name": "RNA-binding protein 15",
  "gene": "UniProtKB:Q96T37",
  "gene_symbol": "RBM15",
  "term_label": "nucleus",
  "term_id": "GO:0005634"
}